{
  "gene": "UniProtKB:Q13112",
  "term_label": "CAF-1 complex",
  "gene_symbol": "CHAF1B",
  "term_id": "GO:0033186",
  "gene_name": "Chromatin assembly factor 1 subunit B"
}